{
  "term_label": "protein tyrosine phosphatase activity",
  "gene_symbol": "PTPRR",
  "gene": "UniProtKB:Q15256",
  "term_id": "GO:0004725",
  "gene_name": "Receptor-type tyrosine-protein phosphatase R"
}